vesicle targeting, to, from or within Golgi [GO:0048199] (biological process) References: PMID:10219233 Sources: GOC:jid, GOC:mah, ISBN:0716731363 Regulation: regulated by regulation of vesicle targeting, to, from or within Golgi [GO:0048209] Relationships: is a type of GO:0006903; is part of Golgi vesicle transport [GO:0048193] Definition: The process in which vesicles are directed to specific destination membranes during transport to, from or within the Golgi apparatus; mediated by the addition of specific coat proteins, including COPI and COPII proteins and clathrin, to the membrane during vesicle formation. Subtypes: GO:0048203, vesicle targeting, inter-Golgi cisterna [GO:0048204], vesicle targeting, cis-Golgi to rough endoplasmic reticulum [GO:0048206], vesicle targeting, rough ER to cis-Golgi [GO:0048207], vesicle targeting, trans-Golgi to periciliary membrane compartment [GO:0097712] Also known as: Golgi vesicle targeting, dictyosome vesicle targeting, vesicle targeting, to, from or within dictyosome